{
  "term_label": "regulation of hippo signaling",
  "gene_name": "Protein KIBRA",
  "gene": "UniProtKB:Q8IX03",
  "term_id": "GO:0035330",
  "gene_symbol": "WWC1"
}